{
  "term_id": "UNKNOWN:0003",
  "gene_symbol": "FAM90A9",
  "gene": "UniProtKB:A6NNJ1",
  "gene_name": "Putative protein FAM90A9",
  "term_label": "Unknown cellular component"
}